{
  "gene_name": "DDB1- and CUL4-associated factor 13",
  "gene_symbol": "DCAF13",
  "term_label": "maturation of SSU-rRNA from tricistronic rRNA transcript (SSU-rRNA, 5.8S rRNA, LSU-rRNA)",
  "gene": "UniProtKB:Q9NV06",
  "term_id": "GO:0000462"
}